histone H2AK127 ubiquitin ligase activity [GO:0140863] (molecular function) References: PMID:28624371 Definition: Catalysis of the transfer of a ubiquitin molecule to histone 2A at the lysine-127 residue. Note: Note that the residue position corresponds to the canonical human H2A2A histone (UniProtKB:Q6FI13); this residue is only present in vertebrates. Residue 1 is the first residue following removal of the initiating Methionine (Met). Note that each histone is encoded by multiple genes, and sequences may vary across different genes within an organism. Relationships: is a type of histone H2A ubiquitin ligase activity [GO:0141053] Also known as: histone H2A-K127 ubiquitin ligase activity, histone ubiquitin ligase activity (H2A-K127 specific)